{
  "gene_symbol": "GABRB3",
  "term_label": "chloride channel activity",
  "gene_name": "Gamma-aminobutyric acid receptor subunit beta-3",
  "term_id": "GO:0005254",
  "gene": "UniProtKB:P28472"
}